{
  "term_id": "GO:0045236",
  "term_label": "CXCR chemokine receptor binding",
  "gene_name": "C-X-C motif chemokine 13",
  "gene_symbol": "CXCL13",
  "gene": "UniProtKB:O43927"
}